{
  "gene_name": "Large ribosomal subunit protein mL65",
  "term_id": "UNKNOWN:0002",
  "term_label": "Unknown biological process",
  "gene_symbol": "MRPS30",
  "gene": "UniProtKB:Q9NP92"
}